{
  "gene_name": "Voltage-dependent R-type calcium channel subunit alpha-1E",
  "term_label": "neuronal cell body",
  "term_id": "GO:0043025",
  "gene_symbol": "CACNA1E",
  "gene": "UniProtKB:Q15878"
}